{
  "gene_name": "Zinc finger protein 701",
  "gene_symbol": "ZNF701",
  "gene": "UniProtKB:Q9NV72",
  "term_id": "GO:0006357",
  "term_label": "regulation of transcription by RNA polymerase II"
}